cell-matrix adhesion involved in mesendodermal cell migration [GO:0003368] (biological process) Sources: GOC:ascb_2009, GOC:dph, GOC:tb Definition: The binding of a cell to the extracellular matrix that contributes to the directed movement of a mesendodermal cell. Relationships: is a type of cell-matrix adhesion involved in ameboidal cell migration [GO:0003366]; is part of GO:0090134